{
  "gene_name": "TIR domain-containing adapter molecule 1",
  "gene_symbol": "TICAM1",
  "gene": "UniProtKB:Q8IUC6",
  "term_id": "GO:0032481",
  "term_label": "positive regulation of type I interferon production"
}